{
  "term_id": "UNKNOWN:0001",
  "gene_symbol": "VAC14",
  "gene": "UniProtKB:Q08AM6",
  "term_label": "Unknown molecular function",
  "gene_name": "Protein VAC14 homolog"
}